{
  "gene_name": "DNA repair protein REV1",
  "gene_symbol": "REV1",
  "term_label": "deoxycytidyl transferase activity",
  "gene": "UniProtKB:Q9UBZ9",
  "term_id": "GO:0017125"
}